negative regulation of endothelin production [GO:1904471] (biological process) Also known as: down regulation of endothelin secretion, down-regulation of endothelin secretion, downregulation of endothelin secretion, down regulation of EDN1 secretion, down regulation of EDN2 secretion, down regulation of EDN3 secretion, down regulation of endothelin-1 secretion, down regulation of endothelin-2 secretion, down regulation of endothelin-3 secretion, down-regulation of EDN1 secretion, down-regulation of EDN2 secretion, down-regulation of EDN3 secretion, down-regulation of endothelin-1 secretion, down-regulation of endothelin-2 secretion, down-regulation of endothelin-3 secretion, downregulation of EDN1 secretion, downregulation of EDN2 secretion, downregulation of EDN3 secretion, downregulation of endothelin-1 secretion, downregulation of endothelin-2 secretion, downregulation of endothelin-3 secretion, inhibition of EDN1 secretion, inhibition of EDN2 secretion, inhibition of EDN3 secretion, inhibition of endothelin secretion, inhibition of endothelin-1 secretion, inhibition of endothelin-2 secretion, inhibition of endothelin-3 secretion, negative regulation of EDN1 secretion, negative regulation of EDN2 secretion, negative regulation of EDN3 secretion, negative regulation of endothelin secretion, negative regulation of endothelin-1 secretion, negative regulation of endothelin-2 secretion, negative regulation of endothelin-3 secretion Relationships: is a type of negative regulation of cytokine production [GO:0001818]; is_a regulation of endothelin production [GO:1904470]; negatively regulates endothelin production [GO:1990775] References: PMID:15560120 Sources: GOC:TermGenie, GO_REF:0000058 Definition: Any process that stops, prevents or reduces the frequency, rate or extent of endothelin production.